{
  "gene_name": "Arginyl-tRNA--protein transferase 1",
  "gene": "UniProtKB:O95260",
  "gene_symbol": "ATE1",
  "term_label": "proteasomal protein catabolic process",
  "term_id": "GO:0010498"
}